{
  "gene_name": "Nuclear pore complex protein Nup214",
  "term_id": "GO:0006405",
  "gene": "UniProtKB:P35658",
  "term_label": "RNA export from nucleus",
  "gene_symbol": "NUP214"
}